{
  "gene": "UniProtKB:Q10589",
  "term_id": "GO:0051607",
  "gene_symbol": "BST2",
  "gene_name": "Bone marrow stromal antigen 2",
  "term_label": "defense response to virus"
}